{
  "gene_symbol": "SPRR2E",
  "term_label": "Unknown biological process",
  "gene": "UniProtKB:P22531",
  "gene_name": "Small proline-rich protein 2E",
  "term_id": "UNKNOWN:0002"
}